negative regulation of antigen processing and presentation [GO:0002578] (biological process) Definition: Any process that stops, prevents, or reduces the frequency, rate, or extent of antigen processing and presentation. Also known as: down regulation of antigen processing and presentation, down-regulation of antigen processing and presentation, downregulation of antigen processing and presentation, inhibition of antigen processing and presentation Sources: GOC:add Subtypes: GO:0002581, GO:0002584, negative regulation of antigen processing and presentation via MHC class Ib [GO:0002593], negative regulation of dendritic cell antigen processing and presentation [GO:0002605], GO:0002614, negative regulation of macrophage antigen processing and presentation [GO:0002617], GO:0002620, negative regulation of B cell antigen processing and presentation [GO:0002623], negative regulation of T cell antigen processing and presentation [GO:0002626] Relationships: is a type of regulation of antigen processing and presentation [GO:0002577]; is_a GO:0002683; negatively regulates antigen processing and presentation [GO:0019882]